{
  "term_id": "GO:0005788",
  "gene_symbol": "ERLEC1",
  "gene": "UniProtKB:Q96DZ1",
  "term_label": "endoplasmic reticulum lumen",
  "gene_name": "Endoplasmic reticulum lectin 1"
}